cerebellum vasculature development [GO:0061300] (biological process) Sources: GOC:dph Relationships: is a type of GO:0001944 Definition: The process whose specific outcome is the progression of the vasculature of the cerebellum over time, from its formation to the mature structure.